{
  "term_label": "regulation of transcription by RNA polymerase II",
  "gene_symbol": "PROX1",
  "gene_name": "Prospero homeobox protein 1",
  "gene": "UniProtKB:Q92786",
  "term_id": "GO:0006357"
}